regulation of shoot system morphogenesis [GO:1900618] (biological process) Definition: Any process that modulates the frequency, rate or extent of shoot morphogenesis. Relationships: is_a regulation of anatomical structure morphogenesis [GO:0022603]; RO_0002211 GO:0010016 Subtypes: regulation of leaf morphogenesis [GO:1901371] Also known as: regulation of shoot morphogenesis Sources: GOC:TermGenie